{
  "gene_symbol": "GNA12",
  "term_label": "G-protein beta/gamma-subunit complex binding",
  "gene": "UniProtKB:Q03113",
  "gene_name": "Guanine nucleotide-binding protein subunit alpha-12",
  "term_id": "GO:0031683"
}